{
  "gene_symbol": "SETMAR",
  "term_id": "GO:0000793",
  "gene": "UniProtKB:Q53H47",
  "gene_name": "Histone-lysine N-methyltransferase SETMAR",
  "term_label": "condensed chromosome"
}